licodione 2'-O-methyltransferase activity [GO:0030751] (molecular function) Also known as: S-adenosyl-L-methionine:licodione 2'-O-methyltransferase activity Relationships: is a type of GO:0008757 Definition: Catalysis of the reaction: S-adenosyl-L-methionine(1+) + licodione = 2'-O-methyllicodione + S-adenosyl-L-homocysteine + H+. Sources: EC:2.1.1.65, RHEA:18521